{
  "term_label": "antimicrobial humoral immune response mediated by antimicrobial peptide",
  "gene_symbol": "CCL3L1",
  "gene_name": "C-C motif chemokine 3-like 1",
  "term_id": "GO:0061844",
  "gene": "UniProtKB:P16619"
}